{
  "term_id": "GO:0009986",
  "gene_symbol": "ANOS1",
  "gene_name": "Anosmin-1",
  "term_label": "cell surface",
  "gene": "UniProtKB:P23352"
}